{
  "term_label": "BMP signaling pathway",
  "gene_symbol": "RGMB",
  "term_id": "GO:0030509",
  "gene_name": "Repulsive guidance molecule B",
  "gene": "UniProtKB:Q6NW40"
}